proboscis morphogenesis, clypeo-labral disc-derived [GO:0010784] (biological process) Sources: GOC:dph, GOC:tb Definition: The process in which the anatomical structures of the proboscis that are derived from the clypeo-labral disc are generated and organized. Relationships: is a type of post-embryonic animal morphogenesis [GO:0009886]; is part of GO:0007453; is part of proboscis morphogenesis [GO:0048734]